cellular response to sugar-phosphate stress [GO:0036447] (biological process) Subtypes: cellular response to glucose-phosphate stress [GO:0036448] References: PMID:17383224 Sources: GOC:am Also known as: cellular response to presence of non-metabolizable sugars Relationships: is a type of cellular response to chemical stress [GO:0062197] Definition: Any process that results in a change in state or activity of a cell (in terms of movement, secretion, enzyme production, gene expression, etc.) as a result of the accumulation of sugar-phosphate.